negative regulation of anthocyanin biosynthetic process [GO:0031541] (biological process) Definition: Any process that stops, prevents, or reduces the frequency, rate or extent of the chemical reactions and pathways resulting in the formation of anthocyanins. Sources: GOC:mah Also known as: down regulation of anthocyanin biosynthetic process, down-regulation of anthocyanin biosynthetic process, downregulation of anthocyanin biosynthetic process, negative regulation of anthocyanin anabolism, negative regulation of anthocyanin biosynthesis, negative regulation of anthocyanin formation, negative regulation of anthocyanin synthesis, inhibition of anthocyanin biosynthetic process Relationships: is a type of negative regulation of flavonoid biosynthetic process [GO:0009964]; is a type of negative regulation of anthocyanin metabolic process [GO:0031538]; is a type of regulation of anthocyanin biosynthetic process [GO:0031540]; negatively regulates anthocyanin-containing compound biosynthetic process [GO:0009718]